leukotriene-C(4) hydrolase [GO:0002951] (molecular function) Note: The mouse enzyme is specific for leukotriene C(4), while the human enzyme also has considerable activity toward glutathione and oxidized glutathione (cf. EC:3.4.19.13). PMID:9774450 cites that the mouse form of this enzyme failed to measure activity towards glutathione. Relationships: is a type of omega peptidase activity [GO:0008242] References: PMID:9774450 Sources: RHEA:31563 Definition: Catalysis of the reaction leukotriene C(4) + H2O= leukotriene D(4) + L-glutamate.